{
  "gene": "UniProtKB:Q9Y2J4",
  "term_id": "GO:0030334",
  "gene_name": "Angiomotin-like protein 2",
  "gene_symbol": "AMOTL2",
  "term_label": "regulation of cell migration"
}